specification of distal tubule identity [GO:0072084] (biological process) Definition: The process in which the distal tubule of the kidney nephron acquires its identity. Sources: GOC:bf, GOC:mtg_kidney_jan10 Subtypes: specification of pronephric distal tubule identity [GO:0039010], specification of mesonephric distal tubule identity [GO:0061283], specification of metanephric distal tubule identity [GO:0072295] Relationships: is a type of specification of nephron tubule identity [GO:0072081]; is part of distal tubule morphogenesis [GO:0072156]